{
  "term_id": "GO:0043020",
  "gene_symbol": "CYBA",
  "gene_name": "Cytochrome b-245 light chain",
  "gene": "UniProtKB:P13498",
  "term_label": "NADPH oxidase complex"
}